erythropoietin receptor binding [GO:0005128] (molecular function) Definition: Binding to an erythropoietin receptor. Also known as: erythropoietin, erythropoietin receptor ligand Relationships: is a type of cytokine receptor binding [GO:0005126] Sources: GOC:ai